{
  "term_id": "GO:0005829",
  "gene_name": "Dual specificity protein phosphatase 10",
  "gene": "UniProtKB:Q9Y6W6",
  "gene_symbol": "DUSP10",
  "term_label": "cytosol"
}